ER overload response [GO:0006983] (biological process) Definition: The series of molecular signals initiated by the accumulation of normal or misfolded proteins in the endoplasmic reticulum and leading to activation of transcription by NF-kappaB. References: PMID:10390516 Subtypes: detection of endoplasmic reticulum overloading [GO:0002234], positive regulation of autophagy in response to ER overload [GO:0034263] Also known as: EOR, ER-overload response, endoplasmic reticulum overload response, EOR-mediated NF-kappaB activation, EOR-mediated activation of NF-kappaB, positive regulation of NF-kappaB transcription factor activity by EOR, positive regulation of NF-kappaB transcription factor activity by ER overload response Relationships: is a type of ER-nucleus signaling pathway [GO:0006984]; is a type of GO:0034976; is a type of cellular response to biotic stimulus [GO:0071216]